{
  "term_label": "extracellular matrix organization",
  "gene": "UniProtKB:Q9H4F8",
  "gene_name": "SPARC-related modular calcium-binding protein 1",
  "gene_symbol": "SMOC1",
  "term_id": "GO:0030198"
}